{
  "term_id": "GO:0017154",
  "gene_name": "Plexin-B1",
  "term_label": "semaphorin receptor activity",
  "gene": "UniProtKB:O43157",
  "gene_symbol": "PLXNB1"
}